{
  "gene": "UniProtKB:Q6ZU35",
  "gene_symbol": "CRACD",
  "term_label": "negative regulation of barbed-end actin filament capping",
  "gene_name": "Capping protein-inhibiting regulator of actin dynamics",
  "term_id": "GO:2000813"
}